amyloid-beta binding [GO:0001540] (molecular function) Relationships: is a type of amide binding [GO:0033218]; is a type of peptide binding [GO:0042277] Definition: Binding to an amyloid-beta peptide/protein. Also known as: beta-amyloid binding Sources: GOC:hjd